{
  "gene_name": "Sprouty-related, EVH1 domain-containing protein 1",
  "gene_symbol": "SPRED1",
  "term_id": "GO:0019901",
  "gene": "UniProtKB:Q7Z699",
  "term_label": "protein kinase binding"
}